{
  "gene_name": "Maestro heat-like repeat-containing protein family member 7",
  "term_label": "cytoplasm",
  "gene": "UniProtKB:Q68CQ1",
  "term_id": "GO:0005737",
  "gene_symbol": "MROH7"
}